N-acylneuraminate-9-phosphate synthase activity [GO:0047444] (molecular function) Relationships: is_a transferase activity, transferring alkyl or aryl (other than methyl) groups [GO:0016765] Definition: Catalysis of the reaction: H2O + phosphoenolpyruvate + N-acyl-D-mannosamine 6-phosphate = phosphate + N-acylneuraminate 9-phosphate. Also known as: N-acetylneuraminic acid phosphate synthase activity, N-acetylneuraminate 9-phosphate lyase activity, N-acetylneuraminate 9-phosphate sialic acid 9-phosphate synthase activity, N-acetylneuraminate 9-phosphate synthetase activity, N-acylneuraminate-9-phosphate pyruvate-lyase (pyruvate-phosphorylating) activity, phosphoenolpyruvate:N-acyl-D-mannosamine-6-phosphate 1-(2-carboxy-2-oxoethyl)transferase activity, sialic acid 9-phosphate synthetase activity Sources: EC:2.5.1.57